purine nucleobase transmembrane transport [GO:1904823] (biological process) Definition: The process in which a purine nucleobase is transported across a membrane. Sources: GOC:TermGenie, GO_REF:0000069 Relationships: is a type of purine nucleobase transport [GO:0006863]; is a type of GO:0072530 Subtypes: adenine import across plasma membrane [GO:0098702], guanine transmembrane transport [GO:1903716]